{
  "gene_symbol": "STAB2",
  "term_id": "GO:0005041",
  "gene_name": "Stabilin-2",
  "term_label": "low-density lipoprotein particle receptor activity",
  "gene": "UniProtKB:Q8WWQ8"
}